neuron intrinsic apoptotic signaling pathway in response to oxidative stress [GO:0036480] (biological process) Also known as: oxidative stress-induced neuron apoptosis, oxidative stress-induced neuronal apoptosis, neuron apoptosis in response to oxidative stress Definition: The series of molecular signals in which an intracellular signal is conveyed to trigger the apoptotic death of a neuron. The pathway is induced in response to oxidative stress, a state often resulting from exposure to high levels of reactive oxygen species, and ends when the execution phase of apoptosis is triggered. References: PMID:23858059 Sources: GOC:PARL, GOC:bf Regulation: regulated by regulation of oxidative stress-induced neuron intrinsic apoptotic signaling pathway [GO:1903376]; negatively regulated by negative regulation of oxidative stress-induced neuron intrinsic apoptotic signaling pathway [GO:1903377]; positively regulated by positive regulation of oxidative stress-induced neuron intrinsic apoptotic signaling pathway [GO:1903378] Relationships: is a type of intrinsic apoptotic signaling pathway in response to oxidative stress [GO:0008631]; is part of neuron apoptotic process [GO:0051402] Subtypes: neuron intrinsic apoptotic signaling pathway in response to hydrogen peroxide [GO:0036482]